positive regulation of transcription elongation by RNA polymerase I [GO:2001209] (BP) Definition: Any process that activates or increases the frequency, rate or extent of transcription elongation from RNA polymerase I promoter. References: PMID:20299458 Also known as: positive regulation of RNA elongation from Pol I promoter, positive regulation of transcription elongation from RNA polymerase I promoter Relationships: is a type of positive regulation of DNA-templated transcription, elongation [GO:0032786]; is a type of positive regulation of transcription by RNA polymerase I [GO:0045943]; is a type of regulation of transcription elongation by RNA polymerase I [GO:2001207]; positively regulates transcription elongation by RNA polymerase I [GO:0006362]